{
  "term_label": "resolution of meiotic recombination intermediates",
  "term_id": "GO:0000712",
  "gene_symbol": "CENPS",
  "gene_name": "Centromere protein S",
  "gene": "UniProtKB:Q8N2Z9"
}